{
  "term_id": "GO:0005786",
  "gene": "UniProtKB:P37108",
  "term_label": "signal recognition particle, endoplasmic reticulum targeting",
  "gene_name": "Signal recognition particle 14 kDa protein",
  "gene_symbol": "SRP14"
}